{
  "gene": "UniProtKB:Q7RTM1",
  "term_label": "proton transmembrane transport",
  "gene_symbol": "OTOP1",
  "gene_name": "Proton channel OTOP1",
  "term_id": "GO:1902600"
}